{
  "term_label": "positive regulation of apoptotic signaling pathway",
  "gene_name": "Small ribosomal subunit protein uS3",
  "gene_symbol": "RPS3",
  "gene": "UniProtKB:P23396",
  "term_id": "GO:2001235"
}